{
  "term_label": "structural constituent of ribosome",
  "gene_name": "Polyubiquitin-C",
  "gene": "UniProtKB:P0CG48",
  "gene_symbol": "UBC",
  "term_id": "GO:0003735"
}